negative regulation of mitochondrial membrane potential [GO:0010917] (biological process) Relationships: is a type of negative regulation of membrane potential [GO:0045837]; is a type of regulation of mitochondrial membrane potential [GO:0051881] Sources: GOC:dph, GOC:tb Definition: Any process that stops, prevents, or reduces the frequency, rate or extent of establishment or extent of a mitochondrial membrane potential, the electric potential existing across any mitochondrial membrane arising from charges in the membrane itself and from the charges present in the media on either side of the membrane. Also known as: reduction of mitochondrial membrane potential